{
  "term_id": "GO:0005794",
  "gene": "UniProtKB:Q8WTW3",
  "term_label": "Golgi apparatus",
  "gene_name": "Conserved oligomeric Golgi complex subunit 1",
  "gene_symbol": "COG1"
}